RNA cap binding [GO:0000339] (molecular function) Definition: Binding to a 7-methylguanosine (m7G) group or derivative located at the 5' end of an RNA molecule. Relationships: is a type of RNA binding [GO:0003723] Also known as: binding to mRNA cap, mRNA cap binding, snRNA cap binding Sources: GOC:krc Subtypes: RNA 7-methylguanosine cap binding [GO:0000340], RNA trimethylguanosine cap binding [GO:0000341], RNA cap 4 binding [GO:0000342], mRNA cap binding [GO:0098808]